{
  "gene_symbol": "ACP5",
  "gene_name": "Tartrate-resistant acid phosphatase type 5",
  "gene": "UniProtKB:P13686",
  "term_id": "GO:0045453",
  "term_label": "bone resorption"
}